fibroblast growth factor receptor signaling pathway involved in positive regulation of cell proliferation in bone marrow [GO:0035604] (biological process) Relationships: is a type of fibroblast growth factor receptor signaling pathway [GO:0008543]; is part of GO:0071864 Also known as: FGF receptor signaling pathway involved in positive regulation of cell proliferation in bone marrow, FGFR signaling pathway involved in positive regulation of cell proliferation in bone marrow, fibroblast growth factor receptor signalling pathway involved in positive regulation of cell proliferation in bone marrow Definition: The series of molecular signals generated as a consequence of a fibroblast growth factor receptor binding to one of its physiological ligands, which activates or increases the frequency, rate or extent of cell proliferation in the bone marrow. Sources: GOC:yaf